{
  "term_id": "GO:0005856",
  "term_label": "cytoskeleton",
  "gene_symbol": "FHOD1",
  "gene": "UniProtKB:Q9Y613",
  "gene_name": "FH1_FH2 domain-containing protein 1"
}